{
  "gene": "UniProtKB:C9J069",
  "gene_name": "Apical junction component 1 homolog",
  "term_id": "GO:0045216",
  "term_label": "cell-cell junction organization",
  "gene_symbol": "AJM1"
}